{
  "gene": "UniProtKB:Q8WUM0",
  "term_label": "nuclear pore outer ring",
  "gene_name": "Nuclear pore complex protein Nup133",
  "gene_symbol": "NUP133",
  "term_id": "GO:0031080"
}